pre-replicative complex assembly involved in cell cycle DNA replication [GO:1902299] (biological process) Sources: GOC:TermGenie, GOC:mtg_cell_cycle Also known as: pre-RC assembly involved in cell cycle DNA replication, pre-replication complex assembly involved in cell cycle DNA replication Relationships: is a type of GO:0022402; is a type of pre-replicative complex assembly [GO:0036388]; is part of cell cycle DNA replication [GO:0044786] Definition: Any pre-replicative complex assembly that is involved in cell cycle DNA replication. Subtypes: GO:0006267, GO:0036390